PTEX complex [GO:0097619] (cellular component) Also known as: Plasmodium translocon of exported proteins References: PMID:19536257, PMID:25043010, PMID:25043043 Sources: GOC:pr Relationships: is a type of membrane protein complex [GO:0098796]; is part of symbiont-containing vacuole membrane [GO:0020005] Definition: A protein complex that acts as a protein trafficking machinery and is responsible for the export of proteins across the parasitophorous (symbiont-containing) vacuolar membrane and into the human host cell. The PTEX complex is located in the vacuole membrane. It is ATP-powered, and comprises heat shock protein 101 (HSP101; a ClpA/B-like ATPase from the AAA+ superfamily, of a type commonly associated with protein translocons), a parasite protein termed PTEX150, and exported protein 2 (EXP2). EXP2 is the potential channel, as it is the membrane-associated component of the core PTEX complex. Two other proteins, PTEX88 and thioredoxin 2 (TRX2), were also identified as PTEX components.